{
  "term_label": "Unknown biological process",
  "term_id": "UNKNOWN:0002",
  "gene_symbol": "MRPS15",
  "gene": "UniProtKB:P82914",
  "gene_name": "Small ribosomal subunit protein uS15m"
}